neuromuscular junction development, skeletal muscle fiber [GO:0098529] (biological process) Relationships: is a type of neuromuscular junction development [GO:0007528]; is part of GO:0048741 Definition: A process that is carried out at the cellular level which results in the assembly, arrangement of constituent parts, or disassembly of a neuromuscular junction that targets a skeletal muscle fiber. Sources: GOC:mtg_OBO2OWL_2013